{
  "term_label": "endothelial cell migration",
  "gene_symbol": "LPXN",
  "gene_name": "Leupaxin",
  "gene": "UniProtKB:O60711",
  "term_id": "GO:0043542"
}